{
  "gene_name": "Protein broad-minded",
  "term_label": "Unknown cellular component",
  "term_id": "UNKNOWN:0003",
  "gene_symbol": "TBC1D32",
  "gene": "UniProtKB:Q96NH3"
}